{
  "gene_symbol": "TRIM67",
  "term_label": "cytoplasm",
  "term_id": "GO:0005737",
  "gene_name": "Tripartite motif-containing protein 67",
  "gene": "UniProtKB:Q6ZTA4"
}